{
  "term_id": "UNKNOWN:0003",
  "gene_symbol": "A0A0G2JQZ4",
  "gene": "UniProtKB:A0A0G2JQZ4",
  "gene_name": "Uncharacterized protein",
  "term_label": "Unknown cellular component"
}